{
  "gene": "UniProtKB:Q8NGG6",
  "gene_symbol": "OR8B12",
  "term_id": "GO:0004984",
  "gene_name": "Olfactory receptor 8B12",
  "term_label": "olfactory receptor activity"
}